{
  "gene_name": "Catenin alpha-1",
  "gene_symbol": "CTNNA1",
  "gene": "UniProtKB:P35221",
  "term_id": "GO:0051015",
  "term_label": "actin filament binding"
}